{
  "gene": "UniProtKB:Q05932",
  "gene_name": "Folylpolyglutamate synthase, mitochondrial",
  "term_label": "cytosol",
  "term_id": "GO:0005829",
  "gene_symbol": "FPGS"
}